{
  "term_id": "GO:0030953",
  "gene": "UniProtKB:O75410",
  "gene_name": "Transforming acidic coiled-coil-containing protein 1",
  "term_label": "astral microtubule organization",
  "gene_symbol": "TACC1"
}